arabitol transmembrane transporter activity [GO:0015167] (molecular function) Definition: Enables the transfer of an arabitol from one side of a membrane to the other. Arabitol is the pentitol derived from arabinose or lyxose by reduction of the aldehyde group. The D enantiomer is present in lichens and mushrooms. Relationships: is a type of carbohydrate transmembrane transporter activity [GO:0015144]; is a type of GO:0015166; BFO_0000050 GO:0015792 Sources: ISBN:0198506732 Also known as: arabinitol transporter activity